{
  "term_label": "RNA polymerase II cis-regulatory region sequence-specific DNA binding",
  "gene_symbol": "ZSCAN16",
  "term_id": "GO:0000978",
  "gene": "UniProtKB:Q9H4T2",
  "gene_name": "Zinc finger and SCAN domain-containing protein 16"
}